{
  "term_label": "Unknown molecular function",
  "gene_symbol": "AMIGO1",
  "gene": "UniProtKB:Q86WK6",
  "gene_name": "Amphoterin-induced protein 1",
  "term_id": "UNKNOWN:0001"
}